{
  "gene_symbol": "RGS9BP",
  "gene_name": "Regulator of G-protein signaling 9-binding protein",
  "term_id": "GO:0050908",
  "term_label": "detection of light stimulus involved in visual perception",
  "gene": "UniProtKB:Q6ZS82"
}